{
  "term_id": "GO:0034599",
  "term_label": "cellular response to oxidative stress",
  "gene": "UniProtKB:Q9UJ68",
  "gene_symbol": "MSRA",
  "gene_name": "Mitochondrial peptide methionine sulfoxide reductase"
}